{
  "gene_symbol": "EFCAB2",
  "term_label": "sperm principal piece",
  "gene": "UniProtKB:Q5VUJ9",
  "term_id": "GO:0097228",
  "gene_name": "Dynein regulatory complex protein 8"
}